{
  "term_id": "GO:0005764",
  "gene_name": "Cathepsin O",
  "gene": "UniProtKB:P43234",
  "gene_symbol": "CTSO",
  "term_label": "lysosome"
}